protein localization to centrosome [GO:0071539] (biological process) Regulation: regulated by GO:1904779; negatively regulated by negative regulation of protein localization to centrosome [GO:1904780]; positively regulated by GO:1904781 Subtypes: GO:0120329, protein localization to pericentriolar material [GO:1905793] Relationships: is a type of GO:1905508 Also known as: protein localisation to centrosome Sources: GOC:ecd Definition: A process in which a protein is transported to, or maintained at, the centrosome.